{
  "term_label": "axoneme",
  "gene_symbol": "BBS1",
  "gene": "UniProtKB:Q8NFJ9",
  "gene_name": "Bardet-Biedl syndrome 1 protein",
  "term_id": "GO:0005930"
}